epithelial cell differentiation involved in salivary gland development [GO:0060690] (biological process) Definition: The process in which a relatively unspecialized cell acquire specialized structural and/or functional features of an epithelial cell of the salivary gland. Subtypes: acinar cell differentiation involved in salivary gland development [GO:0060704] Sources: GOC:dph Relationships: is a type of GO:0030855; is a type of cell differentiation involved in salivary gland development [GO:0060689]